{
  "gene_symbol": "SHANK1",
  "gene_name": "SH3 and multiple ankyrin repeat domains protein 1",
  "term_id": "GO:0035255",
  "term_label": "ionotropic glutamate receptor binding",
  "gene": "UniProtKB:Q9Y566"
}